{
  "term_label": "nucleus",
  "term_id": "GO:0005634",
  "gene_symbol": "RBFOX2",
  "gene_name": "RNA binding protein fox-1 homolog 2",
  "gene": "UniProtKB:O43251"
}